{
  "term_label": "calcium ion binding",
  "gene_name": "Reticulocalbin-3",
  "term_id": "GO:0005509",
  "gene_symbol": "RCN3",
  "gene": "UniProtKB:Q96D15"
}